{
  "term_id": "GO:0005634",
  "gene_symbol": "MAGEA8",
  "gene": "UniProtKB:P43361",
  "gene_name": "Melanoma-associated antigen 8",
  "term_label": "nucleus"
}